{
  "gene_symbol": "GLMP",
  "term_id": "GO:0005764",
  "term_label": "lysosome",
  "gene": "UniProtKB:Q8WWB7",
  "gene_name": "Glycosylated lysosomal membrane protein"
}